{
  "gene_symbol": "PPID",
  "term_id": "GO:0005829",
  "gene_name": "Peptidyl-prolyl cis-trans isomerase D",
  "gene": "UniProtKB:Q08752",
  "term_label": "cytosol"
}